{
  "term_id": "GO:1904315",
  "gene_name": "Glutamate receptor ionotropic, NMDA 3A",
  "gene": "UniProtKB:Q8TCU5",
  "gene_symbol": "GRIN3A",
  "term_label": "transmitter-gated monoatomic ion channel activity involved in regulation of postsynaptic membrane potential"
}